{
  "term_id": "UNKNOWN:0002",
  "gene_name": "Rab5 GDP_GTP exchange factor",
  "gene": "UniProtKB:Q9UJ41",
  "term_label": "Unknown biological process",
  "gene_symbol": "RABGEF1"
}